{
  "term_label": "cytoplasm",
  "gene_symbol": "TNFAIP8L3",
  "gene_name": "Tumor necrosis factor alpha-induced protein 8-like protein 3",
  "term_id": "GO:0005737",
  "gene": "UniProtKB:Q5GJ75"
}